{
  "gene": "UniProtKB:Q8TC92",
  "term_id": "GO:0003756",
  "term_label": "protein disulfide isomerase activity",
  "gene_symbol": "ENOX1",
  "gene_name": "Ecto-NOX disulfide-thiol exchanger 1"
}